dodecyl sulfate metabolic process [GO:0018909] (biological process) Sources: UM-BBD_pathwayID:dds Relationships: is a type of sulfur compound metabolic process [GO:0006790]; is a type of GO:0006805; is a type of GO:0043436 Definition: The chemical reactions and pathways involving dodecyl sulfate, commonly found as sodium dodecyl sulfate (SDS), a component of a variety of synthetic surfactants. Also known as: dodecyl sulfate metabolism, dodecyl sulphate metabolic process, dodecyl sulphate metabolism